{
  "term_id": "UNKNOWN:0001",
  "gene": "UniProtKB:Q8N387",
  "term_label": "Unknown molecular function",
  "gene_symbol": "MUC15",
  "gene_name": "Mucin-15"
}